oxysterol receptor signaling pathway [GO:0141209] (BP) Definition: A nuclear receptor-mediated signaling pathway initiated by an oxysterol binding to an intracellular receptor of the nuclear receptor protein family, and ending with regulation of a downstream cellular process, e.g. transcription. References: PMID:37541371, PMID:9794827 Relationships: is a type of nuclear receptor-mediated steroid hormone signaling pathway [GO:0030518] Also known as: intracellular oxysterol receptor signaling pathway, nuclear receptor-mediated oxysterol signaling pathway